{
  "gene_symbol": "LONP2",
  "gene_name": "Lon protease homolog 2, peroxisomal",
  "gene": "UniProtKB:Q86WA8",
  "term_id": "GO:0005782",
  "term_label": "peroxisomal matrix"
}